{
  "gene_symbol": "RHOJ",
  "term_label": "GTP binding",
  "gene": "UniProtKB:Q9H4E5",
  "gene_name": "Rho-related GTP-binding protein RhoJ",
  "term_id": "GO:0005525"
}